{
  "term_id": "UNKNOWN:0001",
  "term_label": "Unknown molecular function",
  "gene": "UniProtKB:Q96LP2",
  "gene_symbol": "FAM81B",
  "gene_name": "Protein FAM81B"
}